positive regulation of short-term neuronal synaptic plasticity [GO:0048173] (biological process) Also known as: up regulation of short-term neuronal synaptic plasticity, up-regulation of short-term neuronal synaptic plasticity, upregulation of short-term neuronal synaptic plasticity, activation of short-term neuronal synaptic plasticity, stimulation of short-term neuronal synaptic plasticity Note: Note that the syntax of the definition of this term is different from the usual regulation syntax because it describes regulation of a trait rather than regulation of a process. References: PMID:11891290 Sources: GOC:jid Definition: A process that increases short-term neuronal synaptic plasticity, the ability of neuronal synapses to change in the short-term as circumstances require. Short-term neuronal synaptic plasticity generally involves increasing or decreasing synaptic sensitivity. Relationships: is a type of GO:0048172; is a type of GO:0050769